phospholipase C-activating serotonin receptor signaling pathway [GO:0007208] (biological process) Definition: A phospholipase C-activating receptor G protein-coupled receptor signaling pathway initiated by serotonin binding to its receptor on the surface of a target cell, and ending with the regulation of a downstream cellular process, e.g. transcription. Relationships: is_a GO:0007200; is a type of G protein-coupled serotonin receptor signaling pathway [GO:0098664]; has part Gq/11-coupled serotonin receptor activity [GO:0001587] Sources: GOC:dph, GOC:mah, GOC:signaling, GOC:tb Also known as: activation of phospholipase C activity by serotonin receptor signaling pathway, activation of phospholipase C activity by serotonin receptor signalling pathway, serotonin receptor, phospholipase C activating pathway